{
  "gene_symbol": "ING1",
  "gene_name": "Inhibitor of growth protein 1",
  "term_label": "nucleus",
  "term_id": "GO:0005634",
  "gene": "UniProtKB:Q9UK53"
}